{
  "gene_symbol": "GBA3",
  "term_label": "beta-glucosidase activity",
  "term_id": "GO:0008422",
  "gene_name": "Cytosolic beta-glucosidase",
  "gene": "UniProtKB:Q9H227"
}